actinomycin lactonase activity [GO:0047615] (molecular function) Relationships: is a type of carboxylic ester hydrolase activity [GO:0052689] Sources: EC:3.1.1.39, MetaCyc:ACTINOMYCIN-LACTONASE-RXN Definition: Catalysis of the reaction: actinomycin + H2O = actinomycinic monolactone. Also known as: actinomycin lactonohydrolase activity